{
  "gene": "UniProtKB:Q9UQV4",
  "gene_symbol": "LAMP3",
  "term_id": "UNKNOWN:0001",
  "term_label": "Unknown molecular function",
  "gene_name": "Lysosome-associated membrane glycoprotein 3"
}